{
  "gene": "UniProtKB:Q9BZP6",
  "gene_name": "Acidic mammalian chitinase",
  "term_id": "GO:0006032",
  "term_label": "chitin catabolic process",
  "gene_symbol": "CHIA"
}